{
  "term_label": "extracellular space",
  "term_id": "GO:0005615",
  "gene_symbol": "KLK10",
  "gene_name": "Kallikrein-10",
  "gene": "UniProtKB:O43240"
}